peptidyl-serine ADP-deribosylation [GO:0140290] (biological process) Definition: The removal of ADP-ribose from ADP-ribosylserine. References: PMID:28650317, PMID:29234005 Relationships: is a type of protein de-ADP-ribosylation [GO:0051725]